{
  "term_label": "DNA-binding transcription factor activity, RNA polymerase II-specific",
  "gene_name": "LIM_homeobox protein Lhx1",
  "term_id": "GO:0000981",
  "gene_symbol": "LHX1",
  "gene": "UniProtKB:P48742"
}